{
  "gene_symbol": "FGFR2",
  "term_id": "GO:0043235",
  "gene_name": "Fibroblast growth factor receptor 2",
  "term_label": "receptor complex",
  "gene": "UniProtKB:P21802"
}